{
  "gene": "UniProtKB:Q3SYC2",
  "term_label": "triglyceride biosynthetic process",
  "term_id": "GO:0019432",
  "gene_name": "2-acylglycerol O-acyltransferase 2",
  "gene_symbol": "MOGAT2"
}